{
  "term_label": "extracellular space",
  "gene": "UniProtKB:Q9Y493",
  "gene_symbol": "ZAN",
  "term_id": "GO:0005615",
  "gene_name": "Zonadhesin"
}